{
  "gene_symbol": "TXNRD1",
  "gene_name": "Thioredoxin reductase 1, cytoplasmic",
  "gene": "UniProtKB:Q16881",
  "term_id": "GO:0004791",
  "term_label": "thioredoxin-disulfide reductase (NADPH) activity"
}